regulation of exocyst assembly [GO:0001928] (biological process) Note: Note that the assembly is regulated by several small GTPases of the Rab and Rho families. Relationships: is a type of regulation of protein-containing complex assembly [GO:0043254]; is a type of regulation of vesicle docking [GO:0106020]; regulates exocyst assembly [GO:0001927] Sources: GOC:hjd Subtypes: negative regulation of exocyst assembly [GO:0001929], positive regulation of exocyst assembly [GO:0001930] Definition: Any process that modulates the frequency, rate or extent of exocyst assembly.